{
  "term_label": "semaphorin receptor complex",
  "gene_symbol": "PLXNB3",
  "term_id": "GO:0002116",
  "gene_name": "Plexin-B3",
  "gene": "UniProtKB:Q9ULL4"
}